{
  "term_label": "membrane",
  "gene_symbol": "TM4SF4",
  "gene_name": "Transmembrane 4 L6 family member 4",
  "gene": "UniProtKB:P48230",
  "term_id": "GO:0016020"
}